{
  "gene": "UniProtKB:O60784",
  "term_id": "GO:0030276",
  "term_label": "clathrin binding",
  "gene_symbol": "TOM1",
  "gene_name": "Target of Myb1 membrane trafficking protein"
}